{
  "term_label": "regulation of transcription by RNA polymerase II",
  "gene_name": "THAP domain-containing protein 11",
  "term_id": "GO:0006357",
  "gene": "UniProtKB:Q96EK4",
  "gene_symbol": "THAP11"
}